FADH2 binding [GO:0071950] (molecular function) Definition: Binding to the reduced form, FADH2, of flavin-adenine dinucleotide, the coenzyme or the prosthetic group of various flavoprotein oxidoreductase enzymes. Also known as: reduced flavin adenine dinucleotide binding, reduced flavine-adenine dinucleotide binding Relationships: is a type of flavin adenine dinucleotide binding [GO:0050660] Sources: GOC:mah